{
  "gene_name": "Equilibrative nucleoside transporter 4",
  "gene": "UniProtKB:Q7RTT9",
  "term_id": "GO:0005886",
  "gene_symbol": "SLC29A4",
  "term_label": "plasma membrane"
}